{
  "term_id": "UNKNOWN:0002",
  "gene_name": "Probable fibrosin-1",
  "term_label": "Unknown biological process",
  "gene_symbol": "FBRS",
  "gene": "UniProtKB:Q9HAH7"
}